pancreas field specification [GO:0061131] (biological process) Sources: GOC:dph Regulation: positively regulated by GO:0061132 Definition: The process in which a specific region of the gut is delineated into the area in which the pancreas will develop. Relationships: is a type of specification of animal organ identity [GO:0010092]; is part of GO:0061130